{
  "gene_name": "5-hydroxytryptamine receptor 4",
  "gene_symbol": "HTR4",
  "gene": "UniProtKB:Q13639",
  "term_id": "GO:0007198",
  "term_label": "adenylate cyclase-inhibiting serotonin receptor signaling pathway"
}